{
  "term_label": "cell adhesion",
  "gene_name": "Disintegrin and metalloproteinase domain-containing protein 32",
  "term_id": "GO:0007155",
  "gene_symbol": "ADAM32",
  "gene": "UniProtKB:Q8TC27"
}